{
  "term_label": "axon guidance",
  "term_id": "GO:0007411",
  "gene_name": "Neuropilin-1",
  "gene_symbol": "NRP1",
  "gene": "UniProtKB:O14786"
}